{
  "gene_name": "Na(+)_citrate cotransporter",
  "term_id": "GO:0015744",
  "gene_symbol": "SLC13A5",
  "gene": "UniProtKB:Q86YT5",
  "term_label": "succinate transport"
}